{
  "term_id": "GO:0005886",
  "gene": "UniProtKB:Q5SYB0",
  "gene_name": "FERM and PDZ domain-containing protein 1",
  "gene_symbol": "FRMPD1",
  "term_label": "plasma membrane"
}